negative regulation of DNA biosynthetic process [GO:2000279] (biological process) Sources: GOC:obol Definition: Any process that stops, prevents or reduces the frequency, rate or extent of DNA biosynthetic process. Subtypes: negative regulation of telomere maintenance via telomerase [GO:0032211], negative regulation of reverse transcription [GO:1900269], negative regulation of error-prone translesion synthesis [GO:1904332], negative regulation of DNA amplification [GO:1904524] Relationships: is a type of GO:0010558; is a type of negative regulation of DNA metabolic process [GO:0051053]; is a type of regulation of DNA biosynthetic process [GO:2000278]; negatively regulates DNA biosynthetic process [GO:0071897] Also known as: negative regulation of DNA anabolism, negative regulation of DNA biosynthesis, negative regulation of DNA formation, negative regulation of DNA synthesis